{
  "term_id": "UNKNOWN:0001",
  "term_label": "Unknown molecular function",
  "gene": "UniProtKB:A0A286YEX9",
  "gene_symbol": "SCYGR10",
  "gene_name": "Small cysteine and glycine repeat-containing protein 10"
}